{
  "gene": "UniProtKB:Q9Y4C4",
  "term_label": "intracellular signal transduction",
  "gene_symbol": "MFHAS1",
  "gene_name": "Malignant fibrous histiocytoma-amplified sequence 1",
  "term_id": "GO:0035556"
}